D-arabinokinase activity [GO:0047814] (molecular function) Also known as: ATP:D-arabinose 5-phosphotransferase activity, D-arabinokinase (phosphorylating) Definition: Catalysis of the reaction: D-arabinose + ATP = D-arabinose 5-phosphate + ADP. Sources: EC:2.7.1.54, RHEA:24588 Relationships: is a type of kinase activity [GO:0016301]; is a type of phosphotransferase activity, alcohol group as acceptor [GO:0016773]